regulation of cellular response to oxidative stress [GO:1900407] (biological process) Also known as: regulation of adaptive response to oxidative stress Relationships: is a type of regulation of cellular response to stress [GO:0080135]; is_a GO:1902882; regulates cellular response to oxidative stress [GO:0034599] Definition: Any process that modulates the frequency, rate or extent of cellular response to oxidative stress. Subtypes: GO:1900408, positive regulation of cellular response to oxidative stress [GO:1900409], regulation of removal of superoxide radicals [GO:2000121] Sources: GOC:TermGenie, GOC:mah